{
  "term_id": "UNKNOWN:0003",
  "gene": "UniProtKB:Q9UHC7",
  "gene_symbol": "MKRN1",
  "gene_name": "E3 ubiquitin-protein ligase makorin-1",
  "term_label": "Unknown cellular component"
}